{
  "gene_symbol": "NOTCH3",
  "term_label": "receptor complex",
  "gene": "UniProtKB:Q9UM47",
  "gene_name": "Neurogenic locus notch homolog protein 3",
  "term_id": "GO:0043235"
}